{
  "term_id": "GO:0005634",
  "gene_symbol": "ZNF780A",
  "term_label": "nucleus",
  "gene": "UniProtKB:O75290",
  "gene_name": "Zinc finger protein 780A"
}